{
  "gene_symbol": "RHOXF2",
  "gene_name": "Rhox homeobox family member 2",
  "term_label": "RNA polymerase II transcription regulatory region sequence-specific DNA binding",
  "term_id": "GO:0000977",
  "gene": "UniProtKB:Q9BQY4"
}